{
  "gene_name": "Short stature homeobox protein",
  "gene_symbol": "SHOX",
  "term_id": "GO:0005634",
  "term_label": "nucleus",
  "gene": "UniProtKB:O15266"
}